gonadal mesoderm development [GO:0007506] (biological process) Relationships: is_a developmental process involved in reproduction [GO:0003006]; is a type of mesoderm development [GO:0007498]; is a type of mesenchyme development [GO:0060485]; is part of GO:0008406 Sources: GOC:ai Definition: The process whose specific outcome is the progression of the gonadal mesoderm over time, from its formation to the mature structure. The gonadal mesoderm is the middle layer of the three primary germ layers of the embryo which will go on to form the gonads of the organism.